{
  "term_label": "nucleus",
  "gene_name": "Zinc finger and BTB domain-containing protein 7A",
  "gene": "UniProtKB:O95365",
  "gene_symbol": "ZBTB7A",
  "term_id": "GO:0005634"
}